{
  "gene_name": "SH2B adapter protein 3",
  "term_label": "hemopoiesis",
  "gene": "UniProtKB:Q9UQQ2",
  "gene_symbol": "SH2B3",
  "term_id": "GO:0030097"
}